hexuronate:monoatomic cation symporter activity [GO:0015539] (molecular function) Sources: TC:2.A.1.14.2 Definition: Enables the transfer of a solute or solutes from one side of a membrane to the other according to the reaction: hexuronate(out) + cation(out) = hexuronate(in) + cation(in). The hexuronate may be glucuronate or galacturonate. Also known as: hexuronate:cation symporter activity, hexuronate (glucuronate/galacturonate) porter activity, hexuronate porter activity Relationships: is a type of solute:monoatomic cation symporter activity [GO:0015294]; is a type of GO:0046943